methylglyoxal synthase activity [GO:0008929] (molecular function) Sources: EC:4.2.3.3, RHEA:17937 Relationships: is a type of carbon-oxygen lyase activity, acting on phosphates [GO:0016838] Definition: Catalysis of the reaction: glycerone phosphate = methylglyoxal + phosphate. Also known as: glycerone-phosphate phospho-lyase (methylglyoxal-forming), glycerone-phosphate phospho-lyase activity, methylglyoxal synthetase activity